aflatoxin biosynthetic process [GO:0045122] (BP) Relationships: is a type of GO:0006083; is_a GO:0043386; is a type of aflatoxin metabolic process [GO:0046222]; has part fatty-acyl-CoA synthase activity [GO:0004321]; has part versicolorin reductase activity [GO:0042469]; has part versicolorin B synthase activity [GO:0046572]; has part GO:0047145; has part sterigmatocystin 7-O-methyltransferase activity [GO:0047146]; has part norsolorinate anthrone synthase activity [GO:0102973]; has part norsolorinic acid ketoreductase activity [GO:0140393]; has part GO:0140395; has part 5'-hydroxyaverantin dehydrogenase activity [GO:0140396]; has part versiconal hemiacetal acetate esterase activity [GO:0140397]; has part versicolorin B desaturase activity [GO:0140398]; has part aflatoxin B synthase activity [GO:0140399] Also known as: aflatoxin anabolism, aflatoxin biosynthesis, aflatoxin formation, aflatoxin synthesis References: PMID:15006741 Sources: ISBN:0716731363, ISBN:0815316194 Regulation: RO_0002211 by regulation of aflatoxin biosynthetic process [GO:1900177]; RO_0002212 by GO:1900178; positively regulated by positive regulation of aflatoxin biosynthetic process [GO:1900179] Definition: The chemical reactions and pathways resulting in the formation of aflatoxin, a fungal metabolite found as a contaminant in moldy grains that induces liver cancer. Aflatoxin induces a G to T transversion at codon 249 of p53, leading to its inactivation. Aflatoxin is converted to a chemical carcinogen by P450.